axon regeneration [GO:0031103] (biological process) Subtypes: peripheral nervous system axon regeneration [GO:0014012], axon regeneration at neuromuscular junction [GO:0014814], collateral sprouting of intact axon in response to injury [GO:0048673], GO:0101027 Sources: GOC:dgh, GOC:dph, GOC:tb Definition: The regrowth of axons following their loss or damage. Relationships: is a type of GO:0031102; is a type of response to axon injury [GO:0048678]; is a type of GO:0061564 Regulation: regulated by GO:0048679; positively regulated by positive regulation of axon regeneration [GO:0048680]; negatively regulated by negative regulation of axon regeneration [GO:0048681]